cellular response to corticotropin-releasing hormone stimulus [GO:0071376] (biological process) Definition: Any process that results in a change in state or activity of a cell (in terms of movement, secretion, enzyme production, gene expression, etc.) as a result of a corticotropin-releasing hormone stimulus. Corticotropin-releasing hormone is a peptide hormone involved in the stress response. Also known as: cellular response to CRF stimulus, cellular response to CRH stimulus, cellular response to corticoliberin stimulus, cellular response to corticotropin-releasing factor stimulus Relationships: is a type of response to corticotropin-releasing hormone [GO:0043435]; is a type of GO:0071375 Sources: GOC:mah